{
  "gene_symbol": "TBX1",
  "term_id": "GO:0000978",
  "gene_name": "T-box transcription factor TBX1",
  "term_label": "RNA polymerase II cis-regulatory region sequence-specific DNA binding",
  "gene": "UniProtKB:O43435"
}